{
  "term_label": "RNA polymerase II cis-regulatory region sequence-specific DNA binding",
  "term_id": "GO:0000978",
  "gene_name": "Grainyhead-like protein 3 homolog",
  "gene_symbol": "GRHL3",
  "gene": "UniProtKB:Q8TE85"
}